oligopeptide transport [GO:0006857] (biological process) Relationships: is a type of peptide transport [GO:0015833] Regulation: regulated by GO:0090088; negatively regulated by negative regulation of oligopeptide transport [GO:2000877]; positively regulated by positive regulation of oligopeptide transport [GO:2000878] Subtypes: GO:0035672, dipeptide transport [GO:0042938], GO:0042939 Sources: ISBN:0198506732 Definition: The directed movement of oligopeptides into, out of or within a cell, or between cells, by means of some agent such as a transporter or pore. Oligopeptides are molecules that contain a small number (2 to 20) of amino-acid residues connected by peptide linkages.